{
  "gene": "UniProtKB:O00253",
  "gene_symbol": "AGRP",
  "term_id": "GO:0070996",
  "gene_name": "Agouti-related protein",
  "term_label": "type 1 melanocortin receptor binding"
}